{
  "gene": "UniProtKB:O14977",
  "term_label": "ornithine decarboxylase activity",
  "gene_symbol": "AZIN1",
  "term_id": "GO:0004586",
  "gene_name": "Antizyme inhibitor 1"
}